{
  "gene_name": "RNA-binding E3 ubiquitin-protein ligase MEX3C",
  "term_id": "UNKNOWN:0001",
  "gene_symbol": "MEX3C",
  "term_label": "Unknown molecular function",
  "gene": "UniProtKB:Q5U5Q3"
}